{
  "term_label": "Unknown biological process",
  "gene_name": "Zinc finger and BTB domain-containing protein 44",
  "gene_symbol": "ZBTB44",
  "gene": "UniProtKB:Q8NCP5",
  "term_id": "UNKNOWN:0002"
}